saccharopine dehydrogenase (NADP+, L-lysine-forming) activity [GO:0047130] (MF) Also known as: 6-N-(L-1,3-dicarboxypropyl)-L-lysine:NADP+ oxidoreductase (L-lysine-forming), L-lysine-alpha-ketoglutarate reductase activity, N6-(L-1,3-dicarboxypropyl)-L-lysine:NADP+ oxidoreductase (L-lysine-forming), lysine:alpha-ketoglutarate:TPNH oxidoreductase (epsilon-N-[gultaryl-2]-L-lysine forming), saccharopine (nicotinamide adenine dinucleotide phosphate, lysine-forming) dehydrogenase activity Definition: Catalysis of the reaction: L-saccharopine + H2O + NADP+ = 2-oxoglutarate + L-lysine + H+ + NADPH. Sources: EC:1.5.1.8, RHEA:19373 Relationships: is a type of saccharopine dehydrogenase activity [GO:0004753]